{
  "term_label": "chromatin binding",
  "gene_symbol": "SMARCAD1",
  "gene": "UniProtKB:Q9H4L7",
  "gene_name": "SWI_SNF-related matrix-associated actin-dependent regulator of chromatin subfamily A containing DEAD_H box 1",
  "term_id": "GO:0003682"
}